{
  "gene_symbol": "CSTF2",
  "gene_name": "Cleavage stimulation factor subunit 2",
  "term_label": "mRNA cleavage and polyadenylation specificity factor complex",
  "term_id": "GO:0005847",
  "gene": "UniProtKB:P33240"
}